{
  "term_label": "signaling adaptor activity",
  "gene_symbol": "DOK6",
  "term_id": "GO:0035591",
  "gene": "UniProtKB:Q6PKX4",
  "gene_name": "Docking protein 6"
}